cytochrome complex [GO:0070069] (cellular component) Sources: GOC:mah Subtypes: cytochrome o ubiquinol oxidase complex [GO:0009319], cytochrome b6f complex [GO:0009512], respiratory chain complex III [GO:0045275], respiratory chain complex IV [GO:0045277] Definition: A protein complex in which at least one of the proteins is a cytochrome, i.e. a heme-containing protein involved in catalysis of redox reactions. Relationships: is a type of catalytic complex [GO:1902494]